{
  "gene_symbol": "MACIR",
  "term_id": "GO:1900016",
  "term_label": "negative regulation of cytokine production involved in inflammatory response",
  "gene_name": "Macrophage immunometabolism regulator",
  "gene": "UniProtKB:Q96GV9"
}